{
  "gene_name": "Histone acetyltransferase KAT7",
  "gene_symbol": "KAT7",
  "gene": "UniProtKB:O95251",
  "term_id": "GO:0003712",
  "term_label": "transcription coregulator activity"
}